{
  "term_label": "positive regulation of actin filament polymerization",
  "gene": "UniProtKB:Q9UKI2",
  "gene_name": "Cdc42 effector protein 3",
  "gene_symbol": "CDC42EP3",
  "term_id": "GO:0030838"
}